{
  "gene": "UniProtKB:Q8IWB1",
  "term_id": "GO:0004860",
  "gene_name": "Inositol 1,4,5-trisphosphate receptor-interacting protein",
  "term_label": "protein kinase inhibitor activity",
  "gene_symbol": "ITPRIP"
}